melanocyte migration [GO:0097324] (biological process) Definition: The orderly movement of melanocytes from one site to another, often during the development of a multicellular organism. A melanocyte is a pigment cell derived from the neural crest. It contains melanin-filled pigment granules, which give a brown to black appearance. References: PMID:22637532 Sources: CL:0000148, GOC:uh Relationships: is a type of GO:0010631